regulation of tRNA metabolic process [GO:1903326] (biological process) Subtypes: GO:1902370, negative regulation of tRNA metabolic process [GO:1903327], GO:1903328, GO:2000235 Relationships: is a type of regulation of RNA metabolic process [GO:0051252]; regulates GO:0006399 Also known as: regulation of tRNA metabolism Definition: Any process that modulates the frequency, rate or extent of tRNA metabolic process. Sources: GOC:TermGenie, GOC:vw, GO_REF:0000058